{
  "term_label": "Unknown biological process",
  "gene_name": "GTP cyclohydrolase 1 feedback regulatory protein",
  "term_id": "UNKNOWN:0002",
  "gene": "UniProtKB:P30047",
  "gene_symbol": "GCHFR"
}